{
  "term_id": "GO:0031072",
  "term_label": "heat shock protein binding",
  "gene": "UniProtKB:P11021",
  "gene_name": "Endoplasmic reticulum chaperone BiP",
  "gene_symbol": "HSPA5"
}